{
  "gene_name": "Carcinoembryonic antigen-related cell adhesion molecule 18",
  "term_label": "homophilic cell-cell adhesion",
  "term_id": "GO:0007156",
  "gene_symbol": "CEACAM18",
  "gene": "UniProtKB:A8MTB9"
}